{
  "gene": "UniProtKB:Q9UI95",
  "gene_name": "Mitotic spindle assembly checkpoint protein MAD2B",
  "term_label": "DNA repair",
  "term_id": "GO:0006281",
  "gene_symbol": "MAD2L2"
}